neural crest-derived cardiac fibroblast cell fate commitment [GO:0060944] (BP) Sources: GOC:mtg_heart Relationships: is_a cardiac fibroblast cell fate commitment [GO:0060937]; is part of neural crest-derived cardiac fibroblast cell differentiation [GO:0060942] Definition: The commitment of neural crest cells to a cardiac fibroblast fate and their capacity to differentiate into cardiac fibroblast cells. A cardiac fibroblast is a connective tissue cell in the heart which secretes an extracellular matrix rich in collagen and other macromolecules.